negative regulation of granulocyte colony-stimulating factor production [GO:0071656] (biological process) Definition: Any process that stops, prevents, or reduces the frequency, rate, or extent of production of granulocyte colony stimulating factor. Relationships: is a type of GO:0071655; is a type of negative regulation of macrophage colony-stimulating factor production [GO:1901257]; RO_0002212 granulocyte colony-stimulating factor production [GO:0071611] Sources: GOC:mah Also known as: negative regulation of CSF3 production, negative regulation of G-CSF production, negative regulation of colony stimulating factor 3 (granulocyte) production, negative regulation of filgrastim production, negative regulation of granulocyte colony stimulating factor production, negative regulation of lenograstim production, negative regulation of pluripoietin production